{
  "term_label": "G protein-coupled receptor signaling pathway",
  "gene_name": "Regulator of G-protein signaling 11",
  "gene_symbol": "RGS11",
  "term_id": "GO:0007186",
  "gene": "UniProtKB:O94810"
}